{
  "gene": "UniProtKB:A6NFE3",
  "gene_symbol": "EFCAB10",
  "gene_name": "EF-hand calcium-binding domain-containing protein 10",
  "term_label": "Unknown cellular component",
  "term_id": "UNKNOWN:0003"
}